{
  "gene_symbol": "TCEAL4",
  "term_id": "UNKNOWN:0001",
  "gene": "UniProtKB:Q96EI5",
  "gene_name": "Transcription elongation factor A protein-like 4",
  "term_label": "Unknown molecular function"
}